{
  "term_label": "cytoplasm",
  "gene": "UniProtKB:Q9UGV2",
  "term_id": "GO:0005737",
  "gene_symbol": "NDRG3",
  "gene_name": "Protein NDRG3"
}